{
  "gene": "UniProtKB:Q92543",
  "gene_name": "Sorting nexin-19",
  "term_label": "Unknown cellular component",
  "term_id": "UNKNOWN:0003",
  "gene_symbol": "SNX19"
}